corticotropin secretion [GO:0051458] (biological process) Definition: The regulated release of corticotropin by a cell. Corticotropin hormone is a polypeptide hormone synthesized and secreted from corticotropes in the anterior lobe of the pituitary gland in response to corticotropin-releasing hormone (CRH) released by the hypothalamus. References: PMID:11027914 Sources: GOC:cjm Also known as: ACTH secretion, adrenocorticotropic hormone secretion, adrenotropic hormone secretion, adrenotropin secretion, corticotropic hormone secretion, adrenocorticotropin secretion Relationships: is a type of peptide hormone secretion [GO:0030072]; is a type of endocrine hormone secretion [GO:0060986] Regulation: regulated by regulation of corticotropin secretion [GO:0051459]; negatively regulated by negative regulation of corticotropin secretion [GO:0051460]; positively regulated by positive regulation of corticotropin secretion [GO:0051461]